{
  "gene_symbol": "FZD3",
  "gene": "UniProtKB:Q9NPG1",
  "gene_name": "Frizzled-3",
  "term_label": "Wnt receptor activity",
  "term_id": "GO:0042813"
}